{
  "term_label": "axon",
  "term_id": "GO:0030424",
  "gene_symbol": "SEMA3A",
  "gene": "UniProtKB:Q14563",
  "gene_name": "Semaphorin-3A"
}